{
  "term_label": "plasma membrane",
  "term_id": "GO:0005886",
  "gene": "UniProtKB:Q53GD3",
  "gene_symbol": "SLC44A4",
  "gene_name": "Choline transporter-like protein 4"
}